{
  "term_id": "GO:1901052",
  "gene_name": "Glycine N-methyltransferase",
  "gene": "UniProtKB:Q14749",
  "term_label": "sarcosine metabolic process",
  "gene_symbol": "GNMT"
}